{
  "term_id": "GO:0046525",
  "gene_symbol": "B4GALT7",
  "term_label": "xylosylprotein 4-beta-galactosyltransferase activity",
  "gene": "UniProtKB:Q9UBV7",
  "gene_name": "Beta-1,4-galactosyltransferase 7"
}